{
  "gene_name": "Receptor-type tyrosine-protein phosphatase S",
  "term_id": "GO:0007165",
  "gene": "UniProtKB:Q13332",
  "gene_symbol": "PTPRS",
  "term_label": "signal transduction"
}